{
  "gene": "UniProtKB:Q5SZJ8",
  "term_id": "GO:0045666",
  "term_label": "positive regulation of neuron differentiation",
  "gene_name": "BEN domain-containing protein 6",
  "gene_symbol": "BEND6"
}